photosynthetic electron transport chain [GO:0009767] (biological process) Relationships: is a type of GO:0022900; is part of GO:0019684 Definition: A process, occurring as part of photosynthesis, in which light provides the energy for a series of electron carriers to operate together to transfer electrons and generate a transmembrane electrochemical gradient. Also known as: electron carrier, chlorophyll electron transport system, photosynthetic electron transport in cytochrome b6/f, photosynthetic electron transport in plastocyanin, photosynthetic electron transport in plastoquinone Regulation: negatively regulated by photoinhibition [GO:0010205] Subtypes: photosynthetic electron transport in photosystem II [GO:0009772], photosynthetic electron transport in photosystem I [GO:0009773] Sources: GOC:mtg_electron_transport, ISBN:0198547684